exit from diapause [GO:0071981] (biological process) Subtypes: dauer exit [GO:0043054], exit from reproductive diapause [GO:0071983] Definition: The dormancy process that results in exit from diapause. Diapause is a neurohormonally mediated, dynamic state of low metabolic activity. Associated characteristics of this form of dormancy include reduced morphogenesis, increased resistance to environmental extremes, and altered or reduced behavioral activity. Full expression develops in a species-specific manner, usually in response to a number of environmental stimuli that precede unfavorable conditions. Once diapause has begun, metabolic activity is suppressed even if conditions favorable for development prevail. Once initiated, only certain stimuli are capable of releasing the organism from this state, and this characteristic is essential in distinguishing diapause from hibernation. Sources: GOC:mah Relationships: is_a dormancy process [GO:0022611]